{
  "gene_symbol": "HIP1R",
  "gene_name": "Huntingtin-interacting protein 1-related protein",
  "term_id": "GO:0030864",
  "gene": "UniProtKB:O75146",
  "term_label": "cortical actin cytoskeleton"
}